{
  "term_id": "GO:0004326",
  "term_label": "tetrahydrofolylpolyglutamate synthase activity",
  "gene_symbol": "FPGS",
  "gene_name": "Folylpolyglutamate synthase, mitochondrial",
  "gene": "UniProtKB:Q05932"
}